{
  "term_id": "GO:0050766",
  "term_label": "positive regulation of phagocytosis",
  "gene": "UniProtKB:P31995",
  "gene_name": "Low affinity immunoglobulin gamma Fc region receptor II-c",
  "gene_symbol": "FCGR2C"
}